{
  "term_id": "GO:0005654",
  "gene_symbol": "ASH1L",
  "gene": "UniProtKB:Q9NR48",
  "gene_name": "Histone-lysine N-methyltransferase ASH1L",
  "term_label": "nucleoplasm"
}